establishment of pole plasm mRNA localization [GO:0046595] (biological process) Definition: Any process that results in the directed movement of mRNA to the oocyte pole plasm. Sources: GOC:bf Also known as: establishment of oocyte pole plasm mRNA localization, establishment of pole plasm mRNA localisation Relationships: is a type of establishment of RNA localization [GO:0051236]; is a type of establishment of localization in cell [GO:0051649]; is part of pole plasm mRNA localization [GO:0019094]